proacrosomal vesicle fusion [GO:0120211] (biological process) Relationships: is a type of vesicle fusion [GO:0006906]; is part of acrosome assembly [GO:0001675] References: PMID:29991750 Sources: GOC:krc Definition: Fusion of the membrane of proacrosomal vesicle with the membrane of another proacrosomal vesicle to form the acrosome.